{
  "term_id": "GO:0005783",
  "gene_symbol": "P3H3",
  "term_label": "endoplasmic reticulum",
  "gene_name": "Prolyl 3-hydroxylase 3",
  "gene": "UniProtKB:Q8IVL6"
}